{
  "term_id": "UNKNOWN:0002",
  "gene_symbol": "CPSF1",
  "term_label": "Unknown biological process",
  "gene_name": "Cleavage and polyadenylation specificity factor subunit 1",
  "gene": "UniProtKB:Q10570"
}